guanylylpyridinol adenylase activity [GO:0160301] (molecular function) References: PMID:25882909 Relationships: is a type of GO:0016779 Definition: Catalysis of the reaction: guanylylpyridinol + ATP + H+ = guanylylpyridinol-AMP + diphosphate.